positive regulation of fatty acid biosynthetic process [GO:0045723] (biological process) Sources: GOC:go_curators Subtypes: positive regulation of butyryl-CoA biosynthetic process from acetyl-CoA [GO:1900496], positive regulation of butyryl-CoA catabolic process to butyrate [GO:1900502], positive regulation of methyl-branched fatty acid biosynthetic process [GO:1902324], positive regulation of unsaturated fatty acid biosynthetic process [GO:2001280] Definition: Any process that activates or increases the frequency, rate or extent of the chemical reactions and pathways resulting in the formation of fatty acids. Relationships: is a type of GO:0042304; is a type of positive regulation of fatty acid metabolic process [GO:0045923]; is a type of positive regulation of lipid biosynthetic process [GO:0046889]; positively regulates GO:0006633 Also known as: positive regulation of fatty acid anabolism, positive regulation of fatty acid biosynthesis, positive regulation of fatty acid formation, positive regulation of fatty acid synthesis, up regulation of fatty acid biosynthetic process, up-regulation of fatty acid biosynthetic process, upregulation of fatty acid biosynthetic process, activation of fatty acid biosynthetic process, stimulation of fatty acid biosynthetic process